{
  "gene": "UniProtKB:Q96R48",
  "term_label": "olfactory receptor activity",
  "term_id": "GO:0004984",
  "gene_symbol": "OR2A5",
  "gene_name": "Olfactory receptor 2A5"
}